{
  "gene": "UniProtKB:Q9NTK5",
  "term_label": "Unknown biological process",
  "term_id": "UNKNOWN:0002",
  "gene_name": "Obg-like ATPase 1",
  "gene_symbol": "OLA1"
}